{
  "gene_name": "Peptidyl-prolyl cis-trans isomerase FKBP11",
  "gene_symbol": "FKBP11",
  "term_id": "UNKNOWN:0002",
  "gene": "UniProtKB:Q9NYL4",
  "term_label": "Unknown biological process"
}